{
  "gene_name": "Protein mono-ADP-ribosyltransferase PARP16",
  "term_id": "GO:0016020",
  "term_label": "membrane",
  "gene": "UniProtKB:Q8N5Y8",
  "gene_symbol": "PARP16"
}